{
  "term_label": "Unknown molecular function",
  "term_id": "UNKNOWN:0001",
  "gene": "UniProtKB:P08247",
  "gene_name": "Synaptophysin",
  "gene_symbol": "SYP"
}